spermatid nucleus elongation [GO:0007290] (biological process) Sources: GOC:bf, GOC:dph, GOC:jl, GOC:mah, ISBN:0879694238 Also known as: spermatid nuclear elongation Definition: The change in shape of the spermatid nucleus from a spherical structure to an elongated organelle, during the latter part of spermatid differentiation. Relationships: is a type of GO:0006997; is part of GO:0007289